regulation of cardiac muscle hypertrophy in response to stress [GO:1903242] (biological process) Definition: Any process that modulates the frequency, rate or extent of cardiac muscle hypertrophy in response to stress. Subtypes: negative regulation of cardiac muscle hypertrophy in response to stress [GO:1903243], positive regulation of cardiac muscle hypertrophy in response to stress [GO:1903244] Relationships: is a type of regulation of cardiac muscle hypertrophy [GO:0010611]; is a type of regulation of cardiac muscle adaptation [GO:0010612]; is a type of regulation of response to stress [GO:0080134]; regulates cardiac muscle hypertrophy in response to stress [GO:0014898] References: PMID:19287093 Sources: GOC:BHF, GOC:TermGenie, GOC:rl, GO_REF:0000058